{
  "gene_symbol": "HTR6",
  "term_label": "adenylate cyclase-modulating G protein-coupled receptor signaling pathway",
  "gene_name": "5-hydroxytryptamine receptor 6",
  "gene": "UniProtKB:P50406",
  "term_id": "GO:0007188"
}